{
  "gene": "UniProtKB:Q9H4I3",
  "term_label": "Unknown biological process",
  "gene_symbol": "TRABD",
  "term_id": "UNKNOWN:0002",
  "gene_name": "TraB domain-containing protein"
}